{
  "gene_name": "Ubiquitin carboxyl-terminal hydrolase 17-like protein 18",
  "term_id": "GO:0031647",
  "term_label": "regulation of protein stability",
  "gene_symbol": "USP17L18",
  "gene": "UniProtKB:D6R9N7"
}